{
  "term_label": "insulin-like growth factor receptor binding",
  "gene_symbol": "IGF1",
  "gene": "UniProtKB:P05019",
  "gene_name": "Insulin-like growth factor I",
  "term_id": "GO:0005159"
}